{
  "term_label": "sarcoplasmic reticulum lumen",
  "term_id": "GO:0033018",
  "gene_name": "Calsequestrin-1",
  "gene": "UniProtKB:P31415",
  "gene_symbol": "CASQ1"
}